{
  "gene_name": "Nuclear transcription factor Y subunit gamma",
  "gene_symbol": "NFYC",
  "gene": "UniProtKB:Q13952",
  "term_id": "GO:0006357",
  "term_label": "regulation of transcription by RNA polymerase II"
}